{
  "term_id": "GO:0051046",
  "gene_name": "Islet cell autoantigen 1",
  "term_label": "regulation of secretion",
  "gene": "UniProtKB:Q05084",
  "gene_symbol": "ICA1"
}